6-hydroxymellein O-methyltransferase activity [GO:0030773] (molecular function) Relationships: is a type of S-adenosylmethionine-dependent methyltransferase activity [GO:0008757] Also known as: 6-hydroxymellein methyltransferase activity, S-adenosyl-L-methionine:6-hydroxymellein 6-O-methyltransferase activity Definition: Catalysis of the reaction: 6-hydroxymellein + S-adenosyl-L-methionine = 6-methoxymellein + S-adenosyl-L-homocysteine + H+. Sources: EC:2.1.1.108, RHEA:15201